L-aspartate transmembrane transporter activity [GO:0015183] (molecular function) Also known as: L-aspartate transporter activity, glutamate/aspartate porter activity, glutamate/aspartate:sodium symporter activity Subtypes: aspartate:glutamate, proton antiporter activity [GO:0000515], L-aspartate:fumarate antiporter activity [GO:0062057] Relationships: is_a GO:0005310; is a type of GO:0015172; is a type of L-amino acid transmembrane transporter activity [GO:0015179]; is_a C4-dicarboxylate transmembrane transporter activity [GO:0015556]; is part of GO:0070778 Definition: Enables the transfer of L-aspartate from one side of a membrane to the other. L-aspartate is the anion derived from aspartic acid. Sources: GOC:go_curators, GOC:mtg_transport, ISBN:0198506732, ISBN:0815340729